stalled replication fork localization to nuclear periphery [GO:0120290] (biological process) References: PMID:33159083 Sources: GOC:krc, GOC:mah Definition: A cellular localization process where a DNA replication fork that has stalled is signaled to relocate and anchor to the nuclear periphery for the time necessary to complete recombination-dependent replication. Relationships: is a type of cellular localization [GO:0051641]; is part of replication fork processing [GO:0031297] Also known as: stalled replication fork localization to nuclear periphery involved in replication fork processing